{
  "gene": "UniProtKB:P07098",
  "gene_symbol": "LIPF",
  "term_label": "triacylglycerol lipase activity",
  "term_id": "GO:0004806",
  "gene_name": "Gastric triacylglycerol lipase"
}